ethanolamine metabolic process [GO:0006580] (biological process) Subtypes: ethanolamine biosynthetic process [GO:0046335], GO:0046336 Sources: ISBN:0192800981 Definition: The chemical reactions and pathways involving ethanolamine (2-aminoethanol), an important water-soluble base of phospholipid (phosphatidylethanolamine). Also known as: ethanolamine metabolism Relationships: is a type of amine metabolic process [GO:0009308]; is a type of GO:0034308